{
  "gene_symbol": "KIF14",
  "term_id": "GO:0005871",
  "gene": "UniProtKB:Q15058",
  "term_label": "kinesin complex",
  "gene_name": "Kinesin-like protein KIF14"
}